{
  "gene": "UniProtKB:O60309",
  "term_label": "Unknown biological process",
  "gene_symbol": "LRRC37A3",
  "gene_name": "Leucine-rich repeat-containing protein 37A3",
  "term_id": "UNKNOWN:0002"
}